aldehyde-lyase activity [GO:0016832] (molecular function) Definition: Catalysis of the cleavage of a C-C bond in a molecule containing a hydroxyl group and a carbonyl group to form two smaller molecules, each being an aldehyde or a ketone. Relationships: is a type of carbon-carbon lyase activity [GO:0016830] Also known as: aldolase activity Sources: GOC:curators Subtypes: deoxyribose-phosphate aldolase activity [GO:0004139], GO:0004150, fructose-bisphosphate aldolase activity [GO:0004332], threonine aldolase activity [GO:0004793], sphinganine-1-phosphate aldolase activity [GO:0008117], 2-dehydro-3-deoxyglucarate aldolase activity [GO:0008672], 2-dehydro-3-deoxy-6-phosphogalactonate aldolase activity [GO:0008674], 2-dehydro-3-deoxy-phosphogluconate aldolase activity [GO:0008675], L-fuculose-phosphate aldolase activity [GO:0008738], rhamnulose-1-phosphate aldolase activity [GO:0008994], tagatose-bisphosphate aldolase activity [GO:0009025], indole-3-glycerol-phosphate lyase activity [GO:0033984], hexulose-6-phosphate synthase activity [GO:0043801], 4-hydroxy-2-ketopimelate aldolase activity [GO:0043863], D-threonine aldolase activity [GO:0043876], GO:0046593, 2-dehydro-3-deoxy-L-pentonate aldolase activity [GO:0047438], 3-deoxy-D-manno-octulosonate aldolase activity [GO:0047439], 2-dehydro-3-deoxy-D-pentonate aldolase activity [GO:0047440], GO:0047441, (S)-hydroxynitrile lyase activity [GO:0047606], benzoin aldolase activity [GO:0047695], GO:0047864, fructose-6-phosphate phosphoketolase activity [GO:0047905], GO:0047906, 2-dehydropantoate aldolase activity [GO:0050013], ketotetrose-phosphate aldolase activity [GO:0050014], lactate aldolase activity [GO:0050041], GO:0050179, phosphoketolase activity [GO:0050193], propioin synthase activity [GO:0050217], trimethylamine-oxide aldolase activity [GO:0050352], hydroxymandelonitrile lyase activity [GO:0050419], GO:0050547, aliphatic (R)-hydroxynitrile lyase activity [GO:0052919], 6-deoxy-6-sulfofructose-1-phosphate aldolase activity [GO:0061595], GO:0061609, 2-dehydro-3-deoxy-D-gluconate aldolase activity [GO:0061677], GO:0097023, GO:0102083, GO:0103042, 2-keto-3-deoxy-L-rhamnonate aldolase activity [GO:0106099], 2-hydroxyacyl-CoA lyase activity [GO:0106359], hydroxytrimethyllysine aldolase activity [GO:0120567]